positive regulation of centriole elongation [GO:1903724] (biological process) Also known as: up regulation of centriole elongation, up-regulation of centriole elongation, upregulation of centriole elongation, activation of centriole elongation Definition: Any process that activates or increases the frequency, rate or extent of centriole elongation. References: PMID:20616062 Sources: GOC:TermGenie, GOC:als, GO_REF:0000058 Relationships: is a type of positive regulation of centriole replication [GO:0046601]; is a type of regulation of centriole elongation [GO:1903722]; RO_0002213 centriole elongation [GO:0061511]